{
  "term_id": "UNKNOWN:0003",
  "gene_name": "Trichohyalin",
  "term_label": "Unknown cellular component",
  "gene": "UniProtKB:Q07283",
  "gene_symbol": "TCHH"
}